{
  "gene": "UniProtKB:Q15361",
  "term_label": "chromatin binding",
  "gene_symbol": "TTF1",
  "term_id": "GO:0003682",
  "gene_name": "Transcription termination factor 1"
}